inosine nucleosidase activity [GO:0047724] (molecular function) Definition: Catalysis of the reaction: inosine + H2O = D-ribose + hypoxanthine. Sources: EC:3.2.2.2, MetaCyc:INOSINE-NUCLEOSIDASE-RXN Also known as: inosinase activity, inosine ribohydrolase activity, inosine-guanosine nucleosidase activity Relationships: is a type of purine nucleosidase activity [GO:0008477]